negative regulation of T cell mediated immune response to tumor cell [GO:0002841] (biological process) Definition: Any process that stops, prevents, or reduces the frequency, rate, or extent of a T cell mediated immune response to tumor cell. Sources: GOC:add Also known as: down regulation of T cell mediated immune response to tumor cell, down-regulation of T cell mediated immune response to tumor cell, downregulation of T cell mediated immune response to tumor cell, negative regulation of T cell mediated immune response to tumour cell, negative regulation of T lymphocyte mediated immune response to tumor cell, negative regulation of T-cell mediated immune response to tumor cell, negative regulation of T-lymphocyte mediated immune response to tumor cell, inhibition of T cell mediated immune response to tumor cell Relationships: is a type of negative regulation of T cell mediated immunity [GO:0002710]; is_a negative regulation of immune response to tumor cell [GO:0002838]; is a type of GO:0002840; negatively regulates T cell mediated immune response to tumor cell [GO:0002424] Subtypes: negative regulation of T cell tolerance induction to tumor cell [GO:0002847], negative regulation of T cell mediated cytotoxicity directed against tumor cell target [GO:0002853]